G protein-coupled serotonin receptor signaling pathway [GO:0098664] (biological process) Sources: GOC:mah Subtypes: adenylate cyclase-inhibiting serotonin receptor signaling pathway [GO:0007198], phospholipase C-activating serotonin receptor signaling pathway [GO:0007208] Also known as: G-protein coupled serotonin receptor signaling pathway Relationships: is a type of G protein-coupled receptor signaling pathway [GO:0007186]; has part G protein-coupled serotonin receptor activity [GO:0004993] Definition: The series of molecular signals generated as a consequence of a G protein-coupled serotonin receptor binding to one of its physiological ligands.